{
  "term_label": "phosphatidylinositol-mediated signaling",
  "gene_name": "Phosphatidylinositol 3-kinase catalytic subunit type 3",
  "gene": "UniProtKB:Q8NEB9",
  "term_id": "GO:0048015",
  "gene_symbol": "PIK3C3"
}